{
  "term_label": "extracellular space",
  "term_id": "GO:0005615",
  "gene_name": "C-C motif chemokine 4-like",
  "gene_symbol": "CCL4L1",
  "gene": "UniProtKB:Q8NHW4"
}